{
  "term_id": "GO:0005829",
  "gene_name": "BH3-interacting domain death agonist",
  "gene_symbol": "BID",
  "gene": "UniProtKB:P55957",
  "term_label": "cytosol"
}